{
  "gene_name": "PDZ and LIM domain protein 4",
  "gene_symbol": "PDLIM4",
  "term_label": "filamentous actin",
  "gene": "UniProtKB:P50479",
  "term_id": "GO:0031941"
}